endodermal cell differentiation [GO:0035987] (biological process) Also known as: endoderm cell differentiation References: PMID:17624332 Sources: CL:0000223, GOC:yaf Definition: The process in which a relatively unspecialized cell acquires the specialized features of an endoderm cell, a cell of the inner of the three germ layers of the embryo. Relationships: is a type of cell differentiation [GO:0030154]; is part of endoderm formation [GO:0001706] Regulation: RO_0002211 by GO:1903224; RO_0002212 by GO:1903225; positively regulated by positive regulation of endodermal cell differentiation [GO:1903226]